{
  "term_id": "GO:0007043",
  "gene_symbol": "CDH6",
  "term_label": "cell-cell junction assembly",
  "gene_name": "Cadherin-6",
  "gene": "UniProtKB:P55285"
}